{
  "term_label": "Unknown biological process",
  "gene_symbol": "MRPS18C",
  "gene": "UniProtKB:Q9Y3D5",
  "term_id": "UNKNOWN:0002",
  "gene_name": "Small ribosomal subunit protein bS18m"
}